{
  "gene_name": "Dolichyldiphosphatase 1",
  "gene": "UniProtKB:Q86YN1",
  "term_id": "GO:0005789",
  "term_label": "endoplasmic reticulum membrane",
  "gene_symbol": "DOLPP1"
}